{
  "term_label": "Unknown molecular function",
  "term_id": "UNKNOWN:0001",
  "gene_symbol": "SNRNP25",
  "gene": "UniProtKB:Q9BV90",
  "gene_name": "U11_U12 small nuclear ribonucleoprotein 25 kDa protein"
}